{
  "term_label": "Unknown cellular component",
  "gene_name": "3-phosphoinositide-dependent protein kinase 1",
  "gene": "UniProtKB:O15530",
  "gene_symbol": "PDPK1",
  "term_id": "UNKNOWN:0003"
}